pyridine nucleoside metabolic process [GO:0070637] (biological process) Relationships: is a type of nucleoside metabolic process [GO:0009116]; is a type of pyridine-containing compound metabolic process [GO:0072524] Subtypes: nicotinamide riboside metabolic process [GO:0046495], pyridine nucleoside catabolic process [GO:0070638], pyridine nucleoside biosynthetic process [GO:0071589] Sources: GOC:mah Definition: The chemical reactions and pathways involving any pyridine nucleoside, a nucleoside in which a pyridine base covalently bonded to a sugar, usually ribose. Also known as: pyridine nucleoside metabolism